{
  "term_id": "GO:0000014",
  "gene_name": "Nuclease EXOG, mitochondrial",
  "term_label": "single-stranded DNA endodeoxyribonuclease activity",
  "gene": "UniProtKB:Q9Y2C4",
  "gene_symbol": "EXOG"
}